{
  "gene": "UniProtKB:Q02880",
  "term_label": "DNA topoisomerase type II (double strand cut, ATP-hydrolyzing) activity",
  "gene_symbol": "TOP2B",
  "gene_name": "DNA topoisomerase 2-beta",
  "term_id": "GO:0003918"
}